regulation of steroid biosynthetic process [GO:0050810] (biological process) Subtypes: GO:0010893, negative regulation of steroid biosynthetic process [GO:0010894], regulation of vitamin D biosynthetic process [GO:0060556], regulation of bile acid biosynthetic process [GO:0070857], GO:0090030, regulation of sterol biosynthetic process [GO:0106118], regulation of helvolic acid biosynthetic process [GO:1900840], GO:1903454, GO:1904076, regulation of progesterone biosynthetic process [GO:2000182], regulation of testosterone biosynthetic process [GO:2000224] Sources: GOC:ai Also known as: regulation of steroid anabolism, regulation of steroid biosynthesis, regulation of steroid formation, regulation of steroid synthesis, regulation of steroidogenesis Relationships: is a type of regulation of steroid metabolic process [GO:0019218]; is a type of regulation of lipid biosynthetic process [GO:0046890]; regulates GO:0006694 Definition: Any process that modulates the frequency, rate or extent of the chemical reactions and pathways resulting in the formation of steroids, compounds with a 1,2,cyclopentanoperhydrophenanthrene nucleus.